{
  "gene": "UniProtKB:Q9H112",
  "gene_symbol": "CST11",
  "term_label": "Unknown molecular function",
  "term_id": "UNKNOWN:0001",
  "gene_name": "Cystatin-11"
}